first spliceosomal transesterification activity [GO:0000384] (molecular function) Relationships: is_a catalytic activity, acting on RNA [GO:0140098]; is part of RNA splicing, via transesterification reactions [GO:0000375] References: PMID:19239890 Sources: GOC:krc, ISBN:0879695897 Definition: Catalysis of the first transesterification reaction of spliceosomal mRNA splicing. The intron branch site adenosine is the nucleophile attacking the 5' splice site, resulting in cleavage at this position. In cis splicing, this is the step that forms a lariat structure of the intron RNA, while it is still joined to the 3' exon. Also known as: lariat formation, 5'-splice site cleavage